{
  "gene_name": "Sentrin-specific protease 2",
  "term_label": "deSUMOylase activity",
  "gene": "UniProtKB:Q9HC62",
  "term_id": "GO:0016929",
  "gene_symbol": "SENP2"
}